{
  "term_id": "GO:0000981",
  "gene": "UniProtKB:Q68DI1",
  "gene_name": "Zinc finger protein 776",
  "gene_symbol": "ZNF776",
  "term_label": "DNA-binding transcription factor activity, RNA polymerase II-specific"
}